{
  "gene": "UniProtKB:Q6P050",
  "term_label": "Unknown cellular component",
  "gene_symbol": "FBXL22",
  "term_id": "UNKNOWN:0003",
  "gene_name": "F-box and leucine-rich protein 22"
}